{
  "gene": "UniProtKB:Q8TAP4",
  "term_id": "GO:0003713",
  "gene_name": "LIM domain only protein 3",
  "term_label": "transcription coactivator activity",
  "gene_symbol": "LMO3"
}